beta-carotene 15,15'-dioxygenase activity [GO:0003834] (molecular function) Relationships: is a type of oxidoreductase activity, acting on single donors with incorporation of molecular oxygen, incorporation of two atoms of oxygen [GO:0016702] Sources: RHEA:32887 Definition: Catalysis of the reaction: all-trans-beta-carotene + O2 = 2 all-trans-retinal. Also known as: beta-carotene 15,15'-monooxygenase activity, carotene 15,15'-dioxygenase activity, carotene dioxygenase activity